cellular response to N-phenylthiourea [GO:1902611] (biological process) References: PMID:24006265 Sources: GOC:TermGenie, GOC:rjd, GO_REF:0000071 Relationships: is a type of GO:0070887; is a type of GO:1902610 Definition: Any process that results in a change in state or activity of a cell (in terms of movement, secretion, enzyme production, gene expression, etc.) as a result of a N-phenylthiourea stimulus.